beta-caryophyllene biosynthetic process [GO:1901937] (biological process) Definition: The chemical reactions and pathways resulting in the formation of beta-caryophyllene. References: PMID:22867794 Sources: GOC:TermGenie Relationships: is a type of sesquiterpene biosynthetic process [GO:0051762] Also known as: beta-caryophyllene anabolism, beta-caryophyllene biosynthesis, beta-caryophyllene formation, beta-caryophyllene synthesis